{
  "term_label": "cytoplasm",
  "gene": "UniProtKB:Q9NVR0",
  "term_id": "GO:0005737",
  "gene_name": "Kelch-like protein 11",
  "gene_symbol": "KLHL11"
}